{
  "gene": "UniProtKB:Q9H939",
  "gene_symbol": "PSTPIP2",
  "term_id": "UNKNOWN:0002",
  "gene_name": "Proline-serine-threonine phosphatase-interacting protein 2",
  "term_label": "Unknown biological process"
}